bile acid and bile salt transport [GO:0015721] (biological process) Subtypes: canalicular bile acid transport [GO:0015722] Definition: The directed movement of bile acid and bile salts into, out of or within a cell, or between cells, by means of some agent such as a transporter or pore. Relationships: is a type of lipid transport [GO:0006869]; is a type of monocarboxylic acid transport [GO:0015718]; is a type of organic hydroxy compound transport [GO:0015850] Also known as: bile acid transport, bile salt transport References: PMID:12663868, PMID:14699511 Sources: GOC:dph, GOC:krc